{
  "term_id": "GO:0005886",
  "term_label": "plasma membrane",
  "gene_name": "Olfactory receptor 52Z1P",
  "gene": "UniProtKB:P0C646",
  "gene_symbol": "OR52Z1P"
}